protein complex involved in cell adhesion [GO:0098636] (cellular component) Also known as: cell adhesion complex Subtypes: integrin complex [GO:0008305], protein complex involved in cell-cell adhesion [GO:0098635], GO:0098637 Definition: Any protein complex that is capable of carrying out some part of the process of cell adhesion to the cell matrix or to another cell. Relationships: is a type of protein-containing complex [GO:0032991] Sources: GOC:dos